{
  "term_label": "neutral L-amino acid transmembrane transporter activity",
  "term_id": "GO:0015175",
  "gene_symbol": "SLC43A2",
  "gene_name": "Large neutral amino acids transporter small subunit 4",
  "gene": "UniProtKB:Q8N370"
}